{
  "gene_symbol": "CTNNB1",
  "term_id": "GO:0060070",
  "gene": "UniProtKB:P35222",
  "term_label": "canonical Wnt signaling pathway",
  "gene_name": "Catenin beta-1"
}